{
  "term_label": "protein desumoylation",
  "gene_symbol": "USPL1",
  "term_id": "GO:0016926",
  "gene_name": "SUMO-specific isopeptidase USPL1",
  "gene": "UniProtKB:Q5W0Q7"
}